{
  "term_label": "cilium assembly",
  "gene": "UniProtKB:Q96NL6",
  "gene_symbol": "SCLT1",
  "gene_name": "Sodium channel and clathrin linker 1",
  "term_id": "GO:0060271"
}